{
  "term_label": "tetrahydrofolate interconversion",
  "gene_name": "C-1-tetrahydrofolate synthase, cytoplasmic",
  "term_id": "GO:0035999",
  "gene_symbol": "MTHFD1",
  "gene": "UniProtKB:P11586"
}